{
  "term_id": "UNKNOWN:0003",
  "term_label": "Unknown cellular component",
  "gene_symbol": "SH2D1A",
  "gene": "UniProtKB:O60880",
  "gene_name": "SH2 domain-containing protein 1A"
}